{
  "gene_name": "Golgin subfamily A member 6B",
  "gene": "UniProtKB:A6NDN3",
  "term_label": "Unknown molecular function",
  "term_id": "UNKNOWN:0001",
  "gene_symbol": "GOLGA6B"
}